positive regulation of skeletal muscle satellite cell differentiation [GO:1902726] (biological process) Also known as: up regulation of satellite cell differentiation, up-regulation of satellite cell differentiation, upregulation of satellite cell differentiation, activation of satellite cell differentiation Definition: Any process that activates or increases the frequency, rate or extent of satellite cell differentiation. References: PMID:23212449 Sources: GOC:TermGenie, GO_REF:0000058 Relationships: is a type of positive regulation of skeletal muscle cell differentiation [GO:2001016]; positively regulates skeletal muscle satellite cell differentiation [GO:0014816]